{
  "gene": "UniProtKB:Q6PUV4",
  "gene_symbol": "CPLX2",
  "gene_name": "Complexin-2",
  "term_label": "synaptic vesicle exocytosis",
  "term_id": "GO:0016079"
}